{
  "term_label": "Unknown cellular component",
  "gene_name": "V-type proton ATPase subunit S1-like protein",
  "gene_symbol": "ATP6AP1L",
  "term_id": "UNKNOWN:0003",
  "gene": "UniProtKB:Q52LC2"
}